{
  "gene": "UniProtKB:Q13952",
  "term_label": "nucleus",
  "term_id": "GO:0005634",
  "gene_name": "Nuclear transcription factor Y subunit gamma",
  "gene_symbol": "NFYC"
}